14-3-3 protein binding [GO:0071889] (molecular function) Definition: Binding to a 14-3-3 protein. A 14-3-3 protein is any of a large family of approximately 30kDa acidic proteins which exist primarily as homo- and heterodimers within all eukaryotic cells, and have been implicated in the modulation of distinct biological processes by binding to specific phosphorylated sites on diverse target proteins, thereby forcing conformational changes or influencing interactions between their targets and other molecules. Each 14-3-3 protein sequence can be roughly divided into three sections: a divergent amino terminus, the conserved core region and a divergent carboxy-terminus. The conserved middle core region of the 14-3-3s encodes an amphipathic groove that forms the main functional domain, a cradle for interacting with client proteins. References: PMID:15167810, PMID:19575580 Sources: GOC:cna, GOC:mah Relationships: is a type of GO:0005515